{
  "term_label": "guanyl-nucleotide exchange factor activity",
  "gene_symbol": "RIN1",
  "gene": "UniProtKB:Q13671",
  "term_id": "GO:0005085",
  "gene_name": "Ras and Rab interactor 1"
}